{
  "term_label": "Unknown molecular function",
  "term_id": "UNKNOWN:0001",
  "gene_name": "EF-hand calcium-binding domain-containing protein 3",
  "gene": "UniProtKB:Q8N7B9",
  "gene_symbol": "EFCAB3"
}